{
  "term_id": "GO:0005634",
  "term_label": "nucleus",
  "gene_name": "RNA binding protein fox-1 homolog 1",
  "gene_symbol": "RBFOX1",
  "gene": "UniProtKB:Q9NWB1"
}